coenzyme A transmembrane transport [GO:0035349] (biological process) Definition: The process in which coenzyme A is transported across a membrane. Coenzyme A, 3'-phosphoadenosine-(5')diphospho(4')pantatheine, is an acyl carrier in many acylation and acyl-transfer reactions in which the intermediate is a thiol ester. Sources: GOC:bf Relationships: is a type of coenzyme A transport [GO:0015880]; is a type of purine-containing compound transmembrane transport [GO:0072530] Subtypes: mitochondrial coenzyme A transmembrane transport [GO:1990559] Note: Note that this term is not intended for use in annotating lateral movement within membranes. Also known as: coenzyme A membrane transport